{
  "term_id": "UNKNOWN:0001",
  "gene_name": "Claudin-22",
  "gene_symbol": "CLDN22",
  "term_label": "Unknown molecular function",
  "gene": "UniProtKB:Q8N7P3"
}